thromboxane A2 receptor activity [GO:0004961] (molecular function) Sources: GOC:signaling, ISBN:0198506732 Definition: Combining with thromboxane A2 (TXA(2)) and transmitting the signal across the membrane to activate an associated G-protein. Relationships: is a type of thromboxane receptor activity [GO:0004960]; is part of thromboxane A2 signaling pathway [GO:0038193] Also known as: TXA(2) receptor activity, TXA2 receptor activity